{
  "gene_name": "Immunoglobulin subtype domain-containing protein",
  "term_label": "transmembrane signaling receptor activity",
  "term_id": "GO:0004888",
  "gene": "UniProtKB:A0A2R8YCY7",
  "gene_symbol": "A0A2R8YCY7"
}